{
  "gene_name": "Izumo sperm-egg fusion protein 2",
  "gene": "UniProtKB:Q6UXV1",
  "term_label": "Unknown molecular function",
  "gene_symbol": "IZUMO2",
  "term_id": "UNKNOWN:0001"
}